{
  "gene_symbol": "TMEM43",
  "gene_name": "Transmembrane protein 43",
  "term_id": "UNKNOWN:0001",
  "term_label": "Unknown molecular function",
  "gene": "UniProtKB:Q9BTV4"
}